{
  "gene_symbol": "TMPRSS11B",
  "term_id": "GO:0016485",
  "gene": "UniProtKB:Q86T26",
  "gene_name": "Transmembrane protease serine 11B",
  "term_label": "protein processing"
}